negative regulation of extracellular exosome assembly [GO:1903552] (biological process) References: PMID:24105262 Sources: GOC:TermGenie, GO_REF:0000058 Relationships: is a type of negative regulation of organelle assembly [GO:1902116]; is a type of GO:1903551; negatively regulates extracellular exosome assembly [GO:0071971] Definition: Any process that stops, prevents or reduces the frequency, rate or extent of extracellular vesicular exosome assembly. Also known as: down regulation of extracellular vesicular exosome assembly, down-regulation of extracellular vesicular exosome assembly, downregulation of extracellular vesicular exosome assembly, negative regulation of extracellular vesicular exosome assembly, inhibition of extracellular vesicular exosome assembly